{
  "gene": "UniProtKB:Q01081",
  "gene_symbol": "U2AF1",
  "term_label": "mRNA splicing, via spliceosome",
  "gene_name": "Splicing factor U2AF 35 kDa subunit",
  "term_id": "GO:0000398"
}